clathrin-dependent endocytosis of virus by host cell [GO:0075512] (biological process) Definition: Any clathrin-mediated endocytosis that is involved in the uptake of a virus into a host cell. Begins by invagination of a specific region of the host cell plasma membrane around the bound virus to form a clathrin-coated pit, which then pinches off to form a clathrin-coated endocytic vesicle containing the virus. Sources: GOC:bf, GOC:jl, VZ:957 Relationships: is a type of receptor-mediated endocytosis of virus by host cell [GO:0019065]; is a type of clathrin-dependent endocytosis [GO:0072583] Also known as: clathrin-mediated endocytosis of virus by host cell, viral penetration via clathrin-mediated endocytosis, viral entry into host cell via clathrin-mediated endocytosis followed by endosome lysis, viral entry into host cell via clathrin-mediated endocytosis